carbamoyl phosphate biosynthetic process [GO:0070409] (biological process) Also known as: carbamoyl phosphate anabolism, carbamoyl phosphate biosynthesis, carbamoyl phosphate formation, carbamoyl phosphate synthesis, carbamyl phosphate biosynthetic process Sources: CHEBI:17672, GOC:mah, GOC:rph Relationships: is a type of carbamoyl phosphate metabolic process [GO:0070408]; is a type of organophosphate biosynthetic process [GO:0090407] Definition: The chemical reactions and pathways resulting in the formation of carbamoyl phosphate, an intermediate in the urea cycle and other nitrogen compound metabolic pathways.